{
  "gene_name": "Chloride intracellular channel protein 3",
  "gene_symbol": "CLIC3",
  "gene": "UniProtKB:O95833",
  "term_id": "GO:0016020",
  "term_label": "membrane"
}